positive regulation of polyamine transmembrane transport [GO:1902269] (biological process) References: PMID:23755272 Sources: GOC:TermGenie Definition: Any process that activates or increases the frequency, rate or extent of polyamine transmembrane transport. Also known as: up regulation of polyamine transmembrane transport, up-regulation of polyamine transmembrane transport, upregulation of polyamine transmembrane transport, activation of polyamine transmembrane transport Relationships: is a type of positive regulation of transmembrane transport [GO:0034764]; is a type of regulation of polyamine transmembrane transport [GO:1902267]; positively regulates GO:1902047